{
  "gene_symbol": "MYF5",
  "gene_name": "Myogenic factor 5",
  "term_label": "regulation of transcription by RNA polymerase II",
  "gene": "UniProtKB:P13349",
  "term_id": "GO:0006357"
}